{
  "gene": "UniProtKB:O60543",
  "term_label": "apoptotic process",
  "term_id": "GO:0006915",
  "gene_name": "Lipid transferase CIDEA",
  "gene_symbol": "CIDEA"
}